U2 snRNP binding [GO:1990447] (molecular function) References: PMID:14713954 Relationships: is a type of GO:0070990 Definition: Binding to a U2 small nuclear ribonucleoprotein particle.